{
  "term_label": "positive regulation of cell migration",
  "gene": "UniProtKB:Q9H3T2",
  "gene_name": "Semaphorin-6C",
  "gene_symbol": "SEMA6C",
  "term_id": "GO:0030335"
}